{
  "term_label": "meiotic attachment of telomere to nuclear envelope",
  "gene_name": "Membrane-anchored junction protein",
  "gene_symbol": "MAJIN",
  "term_id": "GO:0070197",
  "gene": "UniProtKB:Q3KP22"
}